{
  "gene_name": "Immunoglobulin-like and fibronectin type III domain-containing protein 1",
  "gene": "UniProtKB:Q86VF2",
  "gene_symbol": "IGFN1",
  "term_id": "UNKNOWN:0003",
  "term_label": "Unknown cellular component"
}